ossification involved in bone remodeling [GO:0043932] (BP) Relationships: is_a ossification [GO:0001503]; is part of GO:0046849 Sources: GOC:mtg_mpo, GO_REF:0000034 Also known as: ossification involved in bone remodelling Definition: The formation or growth of bone or of a bony substance, or the conversion of fibrous tissue or of cartilage into bone, involved in response to injury or other physical, physiological or environmental stress stimuli.